acetyl-CoA carboxylase activity [GO:0003989] (molecular function) Also known as: acetyl coenzyme A carboxylase activity, acetyl-CoA:carbon-dioxide ligase (ADP-forming) Sources: EC:6.4.1.2 Definition: Catalysis of the reaction: ATP + acetyl-CoA + HCO3- = ADP + phosphate + malonyl-CoA. Relationships: is a type of GO:0016421